{
  "gene_name": "Rho-associated protein kinase 2",
  "gene_symbol": "ROCK2",
  "gene": "UniProtKB:O75116",
  "term_label": "cytoskeleton",
  "term_id": "GO:0005856"
}